{
  "gene_name": "Kinesin-like protein KIF23",
  "gene": "UniProtKB:Q02241",
  "term_label": "cytoplasm",
  "gene_symbol": "KIF23",
  "term_id": "GO:0005737"
}